{
  "gene": "UniProtKB:A6NK02",
  "gene_name": "Tripartite motif-containing protein 75",
  "term_label": "innate immune response",
  "gene_symbol": "TRIM75",
  "term_id": "GO:0045087"
}